{
  "gene_symbol": "FHL1",
  "gene": "UniProtKB:Q13642",
  "gene_name": "Four and a half LIM domains protein 1",
  "term_id": "UNKNOWN:0003",
  "term_label": "Unknown cellular component"
}